{
  "gene": "UniProtKB:Q9P270",
  "gene_name": "SLAIN motif-containing protein 2",
  "gene_symbol": "SLAIN2",
  "term_id": "GO:0007020",
  "term_label": "microtubule nucleation"
}